odorant binding [GO:0005549] (molecular function) Subtypes: pheromone binding [GO:0005550] Sources: GOC:jl, ISBN:0721662544 Relationships: is a type of binding [GO:0005488] Definition: Binding to an odorant, any substance capable of stimulating the sense of smell.